{
  "term_label": "nucleus",
  "gene": "UniProtKB:Q9H4E7",
  "gene_symbol": "DEF6",
  "term_id": "GO:0005634",
  "gene_name": "Differentially expressed in FDCP 6 homolog"
}